regulation of nucleobase-containing compound metabolic process [GO:0019219] (biological process) Relationships: is_a regulation of primary metabolic process [GO:0080090]; regulates GO:0006139 Sources: GOC:go_curators Also known as: regulation of nucleobase, nucleoside, nucleotide and nucleic acid metabolism, regulation of nucleobase, nucleoside, nucleotide and nucleic acid metabolic process Definition: Any cellular process that modulates the frequency, rate or extent of the chemical reactions and pathways involving nucleobases, nucleosides, nucleotides and nucleic acids. Subtypes: regulation of nucleotide metabolic process [GO:0006140], regulation of purine nucleobase metabolic process [GO:0006141], GO:0009118, regulation of transcription, start site selection [GO:0010630], GO:0045934, positive regulation of pyrimidine nucleobase metabolic process [GO:0045985], regulation of acyl-CoA biosynthetic process [GO:0050812], regulation of DNA metabolic process [GO:0051052], regulation of RNA metabolic process [GO:0051252], regulation of coenzyme A biosynthetic process [GO:0080020], regulation of UDP-N-acetylglucosamine biosynthetic process [GO:0106278], GO:1900497, regulation of butyryl-CoA catabolic process to butyrate [GO:1900500], regulation of tetrapyrrole biosynthetic process from glycine and succinyl-CoA [GO:1901413], regulation of isopentenyl diphosphate biosynthetic process, mevalonate pathway [GO:2001210]